{
  "gene": "UniProtKB:Q9HCJ0",
  "term_id": "GO:0000932",
  "gene_name": "Trinucleotide repeat-containing gene 6C protein",
  "term_label": "P-body",
  "gene_symbol": "TNRC6C"
}